lateral line nerve glial cell development [GO:0048937] (BP) Definition: The process aimed at the progression of a lateral line glial cell over time, from initial commitment of the cell to a specific fate, to the fully functional differentiated cell. Sources: GOC:dgh Relationships: is a type of GO:0021782; is part of lateral line nerve glial cell differentiation [GO:0048895] Subtypes: GO:0048939, posterior lateral line nerve glial cell development [GO:0048941]